{
  "gene": "UniProtKB:O43525",
  "gene_name": "Potassium voltage-gated channel subfamily KQT member 3",
  "gene_symbol": "KCNQ3",
  "term_id": "GO:0071805",
  "term_label": "potassium ion transmembrane transport"
}